hair cell differentiation [GO:0035315] (BP) Subtypes: inner ear auditory receptor cell differentiation [GO:0042491], neuromast hair cell differentiation [GO:0048886], vestibular receptor cell differentiation [GO:0060114] Definition: The process in which a relatively unspecialized cell acquires specialized features of a hair cell. Relationships: is a type of epidermal cell differentiation [GO:0009913]; is a type of neuron differentiation [GO:0030182] Sources: GOC:bf